{
  "term_id": "GO:0051015",
  "term_label": "actin filament binding",
  "gene": "UniProtKB:P12883",
  "gene_symbol": "MYH7",
  "gene_name": "Myosin-7"
}